negative regulation of pyloric antrum smooth muscle contraction [GO:0120073] (biological process) Definition: Any process that decreases the frequency, rate or extent of any pyloric antrum smooth muscle contraction. References: PMID:15890336 Sources: GOC:sl Relationships: is a type of GO:0120071; is a type of negative regulation of gastro-intestinal system smooth muscle contraction [GO:1904305]; negatively regulates GO:0120065